{
  "term_id": "UNKNOWN:0003",
  "gene_name": "Suppressor of cytokine signaling 4",
  "term_label": "Unknown cellular component",
  "gene_symbol": "SOCS4",
  "gene": "UniProtKB:Q8WXH5"
}